{
  "term_id": "GO:0141162",
  "gene": "UniProtKB:Q9Y233",
  "gene_name": "cAMP and cAMP-inhibited cGMP 3',5'-cyclic phosphodiesterase 10A",
  "gene_symbol": "PDE10A",
  "term_label": "negative regulation of cAMP/PKA signal transduction"
}